{
  "term_id": "UNKNOWN:0002",
  "gene_name": "Putative inactive neutral ceramidase B",
  "gene_symbol": "ASAH2B",
  "term_label": "Unknown biological process",
  "gene": "UniProtKB:P0C7U1"
}